hyaluronan catabolic process [GO:0030214] (biological process) Definition: The chemical reactions and pathways resulting in the breakdown of hyaluronan, the naturally occurring anionic form of hyaluronic acid. Hyaluronan is a type of non-sulfated glycosaminoglycan composed of the repeating disaccharide unit beta(1,4)-D-glucuronic acid-beta(1,3)-N-acetyl-D-glucosamine. Relationships: is a type of glycosaminoglycan catabolic process [GO:0006027]; is a type of hyaluronan metabolic process [GO:0030212] References: PMID:33171800, PMID:35536932 Also known as: hyaluronan breakdown, hyaluronan catabolism, hyaluronan degradation